serine hydrolase activity [GO:0017171] (molecular function) Sources: Wikipedia:Serine_hydrolase Relationships: is a type of hydrolase activity [GO:0016787] Definition: Catalysis of the hydrolysis of a substrate by a catalytic mechanism that involves a catalytic triad consisting of a serine nucleophile that is activated by a proton relay involving an acidic residue (e.g. aspartate or glutamate) and a basic residue (usually histidine). Subtypes: serine-type peptidase activity [GO:0008236]